{
  "gene_name": "Monocarboxylate transporter 5",
  "gene_symbol": "SLC16A4",
  "term_id": "GO:0005886",
  "gene": "UniProtKB:O15374",
  "term_label": "plasma membrane"
}